diadenylate cyclase activity [GO:0106408] (molecular function) Definition: Catalysis of the reaction: 2 ATP = 3',3'-c-di-AMP + 2 diphosphate. References: PMID:30884174 Sources: RHEA:35655 Also known as: cyclic-di-AMP synthase Relationships: is a type of nucleotidyltransferase activity [GO:0016779]